{
  "gene": "UniProtKB:P02748",
  "term_id": "UNKNOWN:0001",
  "term_label": "Unknown molecular function",
  "gene_name": "Complement component C9",
  "gene_symbol": "C9"
}